{
  "gene_symbol": "PIWIL1",
  "gene": "UniProtKB:Q96J94",
  "gene_name": "Piwi-like protein 1",
  "term_label": "piRNA processing",
  "term_id": "GO:0034587"
}